mature B cell apoptotic process [GO:0002901] (biological process) Relationships: is a type of B cell apoptotic process [GO:0001783]; is part of B cell homeostasis [GO:0001782] Sources: CL:0000785, GOC:add, GOC:mtg_apoptosis, ISBN:0781735149 Regulation: regulated by regulation of mature B cell apoptotic process [GO:0002905]; negatively regulated by GO:0002906; positively regulated by positive regulation of mature B cell apoptotic process [GO:0002907] Definition: Any apoptotic process in a B cell that is mature, having left the bone marrow. Also known as: apoptosis of mature B cells, apoptosis of mature B lymphocytes, apoptosis of mature B-cells, apoptosis of mature B-lymphocytes, mature B cell programmed cell death by apoptosis, mature B lymphocyte apoptosis, mature B lymphocyte programmed cell death by apoptosis, mature B-cell apoptosis, mature B-cell programmed cell death by apoptosis, mature B-lymphocyte apoptosis, mature B-lymphocyte programmed cell death by apoptosis, programmed cell death of mature B cells by apoptosis, programmed cell death of mature B lymphocytes by apoptosis, programmed cell death of mature B-cells by apoptosis, programmed cell death of mature B-lymphocytes by apoptosis, programmed cell death, mature B cells, programmed cell death, mature B lymphocytes, programmed cell death, mature B-cells, programmed cell death, mature B-lymphocytes, mature B cell apoptosis